positive regulation of cardiac chamber formation [GO:1901212] (biological process) Definition: Any process that activates or increases the frequency, rate or extent of cardiac chamber formation. Also known as: activation of heart chamber formation, positive regulation of heart chamber formation, up regulation of cardiac chamber formation, up regulation of heart chamber formation, up-regulation of cardiac chamber formation, up-regulation of heart chamber formation, upregulation of cardiac chamber formation, upregulation of heart chamber formation, activation of cardiac chamber formation Relationships: is a type of regulation of cardiac chamber formation [GO:1901210]; is a type of positive regulation of cardiac chamber morphogenesis [GO:1901221]; positively regulates cardiac chamber formation [GO:0003207] Subtypes: GO:1904944 Sources: GOC:BHF, GOC:TermGenie